{
  "gene_symbol": "GIPR",
  "term_id": "GO:0005886",
  "gene": "UniProtKB:P48546",
  "term_label": "plasma membrane",
  "gene_name": "Gastric inhibitory polypeptide receptor"
}